{
  "gene_symbol": "FCGR2A",
  "gene_name": "Low affinity immunoglobulin gamma Fc region receptor II-a",
  "gene": "UniProtKB:P12318",
  "term_id": "GO:0019864",
  "term_label": "IgG binding"
}